parathyroid gland development [GO:0060017] (BP) Relationships: is a type of gland development [GO:0048732]; is part of endocrine system development [GO:0035270] Sources: GOC:dph, ISBN:0721662544 Definition: The process whose specific outcome is the progression of the parathyroid gland over time, from its formation to the mature structure. The parathyroid gland is an organ specialised for secretion of parathyroid hormone.